{
  "gene_symbol": "AP1B1",
  "term_id": "GO:0016192",
  "term_label": "vesicle-mediated transport",
  "gene": "UniProtKB:Q10567",
  "gene_name": "AP-1 complex subunit beta-1"
}